{
  "gene_name": "Protein WFDC10B",
  "gene": "UniProtKB:Q8IUB3",
  "term_label": "extracellular space",
  "term_id": "GO:0005615",
  "gene_symbol": "WFDC10B"
}